procollagen-proline 4-dioxygenase complex, alpha(III) type [GO:0070388] (cellular component) Relationships: is a type of procollagen-proline 4-dioxygenase complex [GO:0016222] References: PMID:14500733 Definition: A procollagen-proline 4-dioxygenase complex that contains alpha subunits of the type III isoform. Also known as: prolyl 4-hydroxylase complex (alpha(III)-type), procollagen-proline, 2-oxoglutarate-4-dioxygenase complex, alpha(III) type